{
  "term_id": "GO:0030139",
  "gene_symbol": "PLEKHG5",
  "gene": "UniProtKB:O94827",
  "term_label": "endocytic vesicle",
  "gene_name": "Pleckstrin homology domain-containing family G member 5"
}